protein C inhibitor-coagulation factor V complex [GO:0097181] (CC) References: PMID:6323392 Sources: GOC:ans Relationships: is_a serine protease inhibitor complex [GO:0097180] Definition: A heterodimeric protein complex that contains protein C inhibitor (SERPINA5) and coagulation factor V (F5); formation of the complex inhibits the serine protease activity of coagulation factor V. Also known as: PCI-coagulation factor V complex, SERPINA5-coagulation factor V complex, plasma serine protease inhibitor-coagulation factor V complex, protein C inhibitor-F5 complex, serpin A5-coagulation factor V complex